transmembrane receptor protein serine/threonine kinase activity [GO:0004675] (molecular function) Also known as: receptor protein serine/threonine kinase activity, receptor serine/threonine protein kinase activity Sources: RHEA:18673 Definition: Combining with a signal and transmitting the signal from one side of the membrane to the other to initiate a change in cell activity by catalysis of the reaction: ATP protein serine = ADP + protein serine phosphate, and ATP + protein threonine = ADP + protein threonine phosphate. Subtypes: transforming growth factor beta receptor activity [GO:0005024], activin receptor activity [GO:0017002], BMP receptor activity [GO:0098821] Relationships: is a type of protein serine/threonine kinase activity [GO:0004674]; is a type of GO:0019199; is part of GO:0007178